negative regulation of protein localization to cell-cell junction [GO:0150119] (biological process) Definition: Any process that stops, prevents or reduces the frequency, rate or extent of protein localization to cell-cell junction. Relationships: is_a regulation of protein localization to cell-cell junction [GO:0150106]; is a type of negative regulation of protein localization [GO:1903828]; negatively regulates GO:0150105 Also known as: negative regulation of protein localisation to cell-cell junction Subtypes: GO:1904703 Sources: GOC:aruk, GOC:bc